{
  "gene": "UniProtKB:Q9BXW7",
  "term_label": "mitochondrion",
  "term_id": "GO:0005739",
  "gene_symbol": "HDHD5",
  "gene_name": "Haloacid dehalogenase-like hydrolase domain-containing 5"
}